{
  "gene_name": "Heme transporter FLVCR1",
  "term_label": "mitochondrion",
  "gene_symbol": "FLVCR1",
  "term_id": "GO:0005739",
  "gene": "UniProtKB:Q9Y5Y0"
}